{
  "gene_symbol": "RARS1",
  "term_label": "arginyl-tRNA aminoacylation",
  "term_id": "GO:0006420",
  "gene": "UniProtKB:P54136",
  "gene_name": "Arginine--tRNA ligase, cytoplasmic"
}